{
  "gene": "UniProtKB:P33260",
  "gene_name": "Cytochrome P450 2C18",
  "term_label": "epoxygenase P450 pathway",
  "term_id": "GO:0019373",
  "gene_symbol": "CYP2C18"
}